{
  "term_label": "Unknown molecular function",
  "gene_symbol": "FAM200B",
  "gene": "UniProtKB:P0CF97",
  "term_id": "UNKNOWN:0001",
  "gene_name": "Protein FAM200B"
}